{
  "gene_symbol": "SPATA31C2",
  "term_label": "Unknown cellular component",
  "term_id": "UNKNOWN:0003",
  "gene": "UniProtKB:B4DYI2",
  "gene_name": "Putative spermatogenesis-associated protein 31C2"
}